{
  "term_id": "GO:0031118",
  "gene_symbol": "NOP10",
  "gene_name": "H_ACA ribonucleoprotein complex subunit 3",
  "gene": "UniProtKB:Q9NPE3",
  "term_label": "rRNA pseudouridine synthesis"
}